{
  "term_label": "regulation of cell cycle",
  "gene_name": "Baculoviral IAP repeat-containing protein 3",
  "gene": "UniProtKB:Q13489",
  "gene_symbol": "BIRC3",
  "term_id": "GO:0051726"
}